interleukin-1 production [GO:0032612] (biological process) Sources: GOC:mah Relationships: is a type of GO:0001816 Definition: The appearance of interleukin-1 due to biosynthesis or secretion following a cellular stimulus, resulting in an increase in its intracellular or extracellular levels. Also known as: IL-1 production, interleukin-1 biosynthetic process, interleukin-1 secretion Subtypes: interleukin-1 alpha production [GO:0032610], interleukin-1 beta production [GO:0032611] Regulation: regulated by regulation of interleukin-1 production [GO:0032652]; negatively regulated by negative regulation of interleukin-1 production [GO:0032692]; positively regulated by positive regulation of interleukin-1 production [GO:0032732]